{
  "gene_symbol": "KCNA4",
  "term_id": "GO:0043197",
  "gene_name": "Potassium voltage-gated channel subfamily A member 4",
  "term_label": "dendritic spine",
  "gene": "UniProtKB:P22459"
}